positive regulation of mitotic nuclear envelope disassembly [GO:1905559] (biological process) Also known as: positive regulation of mitotic nuclear envelope breakdown, positive regulation of mitotic nuclear envelope catabolism, positive regulation of mitotic nuclear envelope degradation, up regulation of mitotic nuclear envelope breakdown, up regulation of mitotic nuclear envelope catabolism, up regulation of mitotic nuclear envelope degradation, up regulation of mitotic nuclear envelope disassembly, up-regulation of mitotic nuclear envelope breakdown, up-regulation of mitotic nuclear envelope catabolism, up-regulation of mitotic nuclear envelope degradation, up-regulation of mitotic nuclear envelope disassembly, upregulation of mitotic nuclear envelope breakdown, upregulation of mitotic nuclear envelope catabolism, upregulation of mitotic nuclear envelope degradation, upregulation of mitotic nuclear envelope disassembly, activation of mitotic nuclear envelope breakdown, activation of mitotic nuclear envelope catabolism, activation of mitotic nuclear envelope degradation, activation of mitotic nuclear envelope disassembly Definition: Any process that activates or increases the frequency, rate or extent of mitotic nuclear envelope disassembly. References: PMID:18765790 Sources: GOC:TermGenie, GO_REF:0000058 Relationships: is a type of positive regulation of cellular component organization [GO:0051130]; is a type of positive regulation of cell cycle process [GO:0090068]; is a type of regulation of mitotic nuclear envelope disassembly [GO:1905557]; positively regulates mitotic nuclear membrane disassembly [GO:0007077]